{
  "gene": "UniProtKB:Q5TD97",
  "gene_symbol": "FHL5",
  "term_label": "nucleus",
  "term_id": "GO:0005634",
  "gene_name": "Four and a half LIM domains protein 5"
}